{
  "term_label": "autophagosome maturation",
  "gene": "UniProtKB:Q8NHS3",
  "gene_name": "Major facilitator superfamily domain-containing protein 8",
  "gene_symbol": "MFSD8",
  "term_id": "GO:0097352"
}